D4 dopamine receptor binding [GO:0031751] (molecular function) Also known as: D4 dopamine receptor ligand Definition: Binding to a D4 dopamine receptor. Relationships: is_a dopamine receptor binding [GO:0050780] Sources: GOC:mah, GOC:nln